protein transport by the Tat complex [GO:0043953] (biological process) Definition: The process in which folded proteins are transported across cytoplasmic membranes of bacteria and membranes of organelles derived from bacteria (chloroplasts and mitochondria) by the TAT complex. Sources: GOC:pamgo_curators Also known as: twin-arginine translocation pathway, protein secretion by the TAT complex, protein translocation by the TAT complex, protein translocation by the twin-arginine translocation complex Note: Note that this term represents an activity and not a cellular structure. Consider also annotating to the cellular structure term 'TAT protein translocation system complex ; GO:0033281'. Note that this term is used for annotation of proteins that compose the transport complex but not the proteins being transported. Relationships: is a type of protein transmembrane transport [GO:0071806]